{
  "term_label": "plasma membrane",
  "gene_symbol": "SIDT1",
  "gene_name": "SID1 transmembrane family member 1",
  "term_id": "GO:0005886",
  "gene": "UniProtKB:Q9NXL6"
}